{
  "gene": "UniProtKB:Q9NSB8",
  "gene_name": "Homer protein homolog 2",
  "term_label": "regulation of synaptic transmission, glutamatergic",
  "gene_symbol": "HOMER2",
  "term_id": "GO:0051966"
}